{
  "gene": "UniProtKB:Q9NVW2",
  "gene_name": "E3 ubiquitin-protein ligase RLIM",
  "gene_symbol": "RLIM",
  "term_id": "GO:0016567",
  "term_label": "protein ubiquitination"
}